{
  "term_id": "UNKNOWN:0003",
  "gene": "UniProtKB:Q9BYC5",
  "gene_name": "Alpha-(1,6)-fucosyltransferase",
  "term_label": "Unknown cellular component",
  "gene_symbol": "FUT8"
}